bud elongation involved in lung branching [GO:0060449] (biological process) Relationships: is a type of GO:0060602; is part of epithelial tube branching involved in lung morphogenesis [GO:0060441] Sources: GOC:dph, GOC:mtg_lung Definition: The process in which a bud in the lung grows out from the point where it is formed.